{
  "term_id": "GO:0030838",
  "term_label": "positive regulation of actin filament polymerization",
  "gene_name": "Uncharacterized protein C15orf62, mitochondrial",
  "gene_symbol": "C15orf62",
  "gene": "UniProtKB:A8K5M9"
}